{
  "gene_symbol": "RNF112",
  "term_id": "GO:0005525",
  "gene_name": "RING finger protein 112",
  "gene": "UniProtKB:Q9ULX5",
  "term_label": "GTP binding"
}